arabinitol transmembrane transport [GO:0015792] (biological process) Sources: ISBN:0198506732 Also known as: arabinitol transport, arabitol transport Definition: The process in which arabitol is transported across a lipid bilayer, from one side of a membrane to the other. Arabitol is the pentitol derived from arabinose or lyxose by reduction of the aldehyde group. The D enantiomer is present in lichens and mushrooms. Relationships: is a type of polyol transmembrane transport [GO:0015791]; is a type of carbohydrate transmembrane transport [GO:0034219]